negative regulation of fertilization [GO:0060467] (biological process) Subtypes: prevention of polyspermy [GO:0060468] Relationships: is a type of regulation of fertilization [GO:0080154]; is_a negative regulation of reproductive process [GO:2000242]; negatively regulates fertilization [GO:0009566] Sources: GOC:dph Definition: Any process that decreases the rate, frequency or extent of fertilization. Fertilization is the union of gametes of opposite sexes during the process of sexual reproduction to form a zygote. It involves the fusion of the gametic nuclei (karyogamy) and cytoplasm (plasmogamy).